{
  "gene_name": "Protein timeless homolog",
  "term_label": "replication fork protection complex",
  "gene_symbol": "TIMELESS",
  "term_id": "GO:0031298",
  "gene": "UniProtKB:Q9UNS1"
}